{
  "gene": "UniProtKB:Q9H9C1",
  "term_id": "GO:0006886",
  "gene_symbol": "VIPAS39",
  "term_label": "intracellular protein transport",
  "gene_name": "Spermatogenesis-defective protein 39 homolog"
}